{
  "gene_name": "WASH complex subunit 1",
  "gene": "UniProtKB:A8K0Z3",
  "gene_symbol": "WASHC1",
  "term_label": "Arp2/3 complex-mediated actin nucleation",
  "term_id": "GO:0034314"
}